inclusion body [GO:0016234] (CC) Definition: A discrete intracellular part formed of aggregated molecules such as proteins or other biopolymers. Subtypes: aggresome [GO:0016235], nuclear inclusion body [GO:0042405], polyhydroxyalkanoate granule [GO:0070088], GO:0097407, fibrillary inclusion [GO:0097408], GO:0097409, hyaline inclusion [GO:0097412], GO:0097413, Lewy body-like hyaline inclusion [GO:0097416], GO:0097417, GO:0097418, GO:0097419, skein-like inclusion [GO:0097420], laminated body [GO:1990011] References: PMID:11121744 Sources: GOC:mah Relationships: is a type of GO:0005622 Also known as: neuronal cytoplasmic inclusion, cellular inclusion